{
  "gene_name": "Small ribosomal subunit protein eS12",
  "gene_symbol": "RPS12",
  "term_label": "cytosolic small ribosomal subunit",
  "term_id": "GO:0022627",
  "gene": "UniProtKB:P25398"
}